{
  "gene_symbol": "BCE1",
  "term_label": "Unknown biological process",
  "gene_name": "Putative protein BCE-1",
  "term_id": "UNKNOWN:0002",
  "gene": "UniProtKB:O60756"
}